{
  "gene_name": "Uroporphyrinogen-III synthase",
  "term_id": "GO:0006780",
  "gene": "UniProtKB:P10746",
  "gene_symbol": "Mgu",
  "term_label": "uroporphyrinogen III biosynthetic process"
}